{
  "gene_symbol": "LINC00299",
  "term_id": "UNKNOWN:0002",
  "gene": "UniProtKB:Q6ZSB3",
  "gene_name": "Putative uncharacterized protein encoded by LINC00299",
  "term_label": "Unknown biological process"
}